{
  "term_label": "interleukin-11 receptor activity",
  "term_id": "GO:0004921",
  "gene_symbol": "IL6R",
  "gene": "UniProtKB:P08887",
  "gene_name": "Interleukin-6 receptor subunit alpha"
}